negative regulation of optic nerve formation [GO:2000596] (biological process) Relationships: is a type of negative regulation of developmental process [GO:0051093]; is a type of regulation of optic nerve formation [GO:2000595]; negatively regulates GO:0021634 Sources: GOC:obol Definition: Any process that stops, prevents or reduces the frequency, rate or extent of optic nerve formation. Also known as: negative regulation of CN II biosynthesis, negative regulation of CN II formation